{
  "term_label": "olfactory receptor activity",
  "gene": "UniProtKB:Q15622",
  "gene_name": "Olfactory receptor 7A5",
  "gene_symbol": "OR7A5",
  "term_id": "GO:0004984"
}